vesicle targeting, rough ER to cis-Golgi [GO:0048207] (biological process) Relationships: is a type of GO:0048199; is part of GO:0006888 Also known as: rough ER to cis-Golgi targeting, rough endoplasmic reticulum to cis-Golgi targeting, vesicle targeting, rough endoplasmic reticulum to cis-Golgi Definition: The process in which vesicles are directed to specific destination membranes during transport from the rough endoplasmic reticulum to the cis-Golgi. References: PMID:10219233 Sources: GOC:jid, GOC:mah, ISBN:0716731363